{
  "term_label": "oligosaccharyltransferase complex",
  "gene_name": "Dolichyl-diphosphooligosaccharide--protein glycosyltransferase subunit 2",
  "term_id": "GO:0008250",
  "gene_symbol": "RPN2",
  "gene": "UniProtKB:P04844"
}